{
  "gene_symbol": "NME6",
  "term_label": "negative regulation of cell growth",
  "term_id": "GO:0030308",
  "gene": "UniProtKB:O75414",
  "gene_name": "Nucleoside diphosphate kinase 6"
}